BCL-2 complex [GO:0097148] (cellular component) Definition: A homodimeric protein complex consisting of BCL-2, a member of the Bcl-2 family of anti- and proapoptotic regulators. References: PMID:14634621 Sources: GOC:bhm, GOC:so Relationships: is a type of Bcl-2 family protein complex [GO:0097136]